{
  "term_label": "protein serine/threonine phosphatase activity",
  "gene_name": "Serine_threonine-protein phosphatase 2A catalytic subunit beta isoform",
  "gene": "UniProtKB:P62714",
  "gene_symbol": "PPP2CB",
  "term_id": "GO:0004722"
}